{
  "gene_symbol": "CAT",
  "gene_name": "Catalase",
  "gene": "UniProtKB:P04040",
  "term_id": "GO:0004096",
  "term_label": "catalase activity"
}